{
  "gene_name": "Forkhead box protein R2",
  "gene": "UniProtKB:Q6PJQ5",
  "term_label": "Unknown biological process",
  "term_id": "UNKNOWN:0002",
  "gene_symbol": "FOXR2"
}